{
  "gene": "UniProtKB:P02730",
  "term_label": "bicarbonate transport",
  "term_id": "GO:0015701",
  "gene_symbol": "SLC4A1",
  "gene_name": "Band 3 anion transport protein"
}